mannose:sodium symporter activity [GO:0140929] (molecular function) Relationships: is a type of carbohydrate:monoatomic cation symporter activity [GO:0005402]; is a type of solute:sodium symporter activity [GO:0015370]; is a type of mannose transmembrane transporter activity [GO:0015578] References: PMID:22212718, PMID:23451068, PMID:24573086 Definition: Enables the transfer of a solute or solutes from one side of a membrane to the other according to the reaction: D-mannose(out) + Na+(out) = D-mannose(in) + Na+(in).